{
  "gene_symbol": "IFT52",
  "gene": "UniProtKB:Q9Y366",
  "term_label": "centriole",
  "term_id": "GO:0005814",
  "gene_name": "Intraflagellar transport protein 52 homolog"
}